{
  "gene_name": "Latent-transforming growth factor beta-binding protein 3",
  "term_label": "transforming growth factor beta receptor signaling pathway",
  "gene_symbol": "LTBP3",
  "gene": "UniProtKB:Q9NS15",
  "term_id": "GO:0007179"
}